{
  "gene_symbol": "BFSP2",
  "term_id": "GO:0005882",
  "term_label": "intermediate filament",
  "gene_name": "Phakinin",
  "gene": "UniProtKB:Q13515"
}